{
  "term_id": "GO:0015813",
  "gene_symbol": "SLC25A18",
  "term_label": "L-glutamate transmembrane transport",
  "gene_name": "Mitochondrial glutamate carrier 2",
  "gene": "UniProtKB:Q9H1K4"
}